{
  "gene_name": "Protein FAM72A",
  "gene": "UniProtKB:Q5TYM5",
  "term_label": "Unknown biological process",
  "term_id": "UNKNOWN:0002",
  "gene_symbol": "FAM72A"
}